{
  "gene_name": "OTU domain-containing protein 3",
  "gene": "UniProtKB:Q5T2D3",
  "term_id": "GO:0004843",
  "term_label": "cysteine-type deubiquitinase activity",
  "gene_symbol": "OTUD3"
}